{
  "gene_name": "Zinc finger protein 233",
  "gene": "UniProtKB:A6NK53",
  "term_label": "Unknown biological process",
  "term_id": "UNKNOWN:0002",
  "gene_symbol": "ZNF233"
}